postsynaptic neurotransmitter receptor cycle [GO:0099630] (biological process) Definition: The process during which neurotransmitter receptors in the postsynaptic specialization membrane are recycled via the endosome. This cycle includes release from anchoring (trapping), diffusion in the synaptic membrane to the postsynaptic endocytic region, endocytosis, transport to the endosome, recycling in the endosome, transport back the synaptic membrane and subsequent trapping in the postsynaptic specialization membrane. Relationships: is a type of establishment of localization in cell [GO:0051649]; is a type of GO:0099627; occurs in GO:0098794 References: PMID:18832033